{
  "term_label": "Unknown molecular function",
  "gene_symbol": "PLK5",
  "gene_name": "Inactive serine_threonine-protein kinase PLK5",
  "term_id": "UNKNOWN:0001",
  "gene": "UniProtKB:Q496M5"
}